{
  "gene_name": "Acyl-coenzyme A thioesterase 8",
  "term_id": "GO:0005782",
  "gene_symbol": "ACOT8",
  "gene": "UniProtKB:O14734",
  "term_label": "peroxisomal matrix"
}